aldose-6-phosphate reductase (NADPH) activity [GO:0047641] (molecular function) Definition: Catalysis of the reaction: D-glucitol 6-phosphate + NADP+ = D-glucose 6-phosphate + H+ + NADPH. Relationships: is a type of GO:0016616 Sources: EC:1.1.1.200, RHEA:20037 Also known as: A6PR, D-aldose-6-phosphate:NADP+ 1-oxidoreductase activity, NADP-dependent D-sorbitol-6-phosphate dehydrogenase activity, NADP-dependent aldose 6-phosphate reductase activity, alditol 6-phosphate:NADP 1-oxidoreductase activity, aldose 6-phosphate reductase activity, aldose-6-P reductase activity, aldose-6-phosphate reductase activity